{
  "gene": "UniProtKB:Q86TW2",
  "gene_name": "AarF domain-containing protein kinase 1",
  "term_id": "GO:0005743",
  "term_label": "mitochondrial inner membrane",
  "gene_symbol": "ADCK1"
}